{
  "gene_name": "Tumor necrosis factor-inducible gene 6 protein",
  "gene": "UniProtKB:P98066",
  "gene_symbol": "TNFAIP6",
  "term_label": "Unknown molecular function",
  "term_id": "UNKNOWN:0001"
}